{
  "term_label": "cytosol",
  "gene_name": "Protein Hikeshi",
  "gene": "UniProtKB:Q53FT3",
  "gene_symbol": "HIKESHI",
  "term_id": "GO:0005829"
}